intracellular magnesium ion homeostasis [GO:0010961] (biological process) Definition: A homeostatic process involved in the maintenance of a steady state level of magnesium ions within a cell. Sources: GOC:dph, GOC:tb Also known as: cellular magnesium ion homeostasis Relationships: is a type of magnesium ion homeostasis [GO:0010960]; is a type of intracellular monoatomic cation homeostasis [GO:0030003]